{
  "gene_symbol": "IGKV2D-24",
  "gene": "UniProtKB:A0A075B6R9",
  "term_label": "Unknown molecular function",
  "term_id": "UNKNOWN:0001",
  "gene_name": "Probable non-functional immunoglobulin kappa variable 2D-24"
}